{
  "gene_symbol": "SNAI1",
  "term_label": "Unknown cellular component",
  "gene_name": "Zinc finger protein SNAI1",
  "term_id": "UNKNOWN:0003",
  "gene": "UniProtKB:O95863"
}